{
  "gene_symbol": "SEMA5B",
  "term_label": "neural crest cell migration",
  "term_id": "GO:0001755",
  "gene": "UniProtKB:Q9P283",
  "gene_name": "Semaphorin-5B"
}